{
  "gene_name": "Rab11 family-interacting protein 5",
  "gene": "UniProtKB:Q9BXF6",
  "term_label": "secretory granule",
  "term_id": "GO:0030141",
  "gene_symbol": "RAB11FIP5"
}